{
  "gene_symbol": "SOX5",
  "gene_name": "Transcription factor SOX-5",
  "gene": "UniProtKB:P35711",
  "term_id": "GO:0000981",
  "term_label": "DNA-binding transcription factor activity, RNA polymerase II-specific"
}